{
  "gene_symbol": "ZNF155",
  "gene": "UniProtKB:Q12901",
  "term_id": "UNKNOWN:0002",
  "term_label": "Unknown biological process",
  "gene_name": "Zinc finger protein 155"
}